{
  "gene_name": "Interleukin-9 receptor",
  "gene_symbol": "IL9R",
  "term_id": "GO:0019983",
  "gene": "UniProtKB:Q01113",
  "term_label": "interleukin-9 binding"
}